{
  "gene_symbol": "AGAP4",
  "gene_name": "Arf-GAP with GTPase, ANK repeat and PH domain-containing protein 4",
  "term_id": "UNKNOWN:0003",
  "gene": "UniProtKB:Q96P64",
  "term_label": "Unknown cellular component"
}